{
  "term_id": "GO:0009098",
  "term_label": "L-leucine biosynthetic process",
  "gene_symbol": "BCAT2",
  "gene": "UniProtKB:O15382",
  "gene_name": "Branched-chain-amino-acid aminotransferase, mitochondrial"
}